{
  "gene": "UniProtKB:P62805",
  "gene_symbol": "H4C16",
  "term_id": "GO:0005634",
  "gene_name": "Histone H4",
  "term_label": "nucleus"
}